{
  "term_label": "lateral element",
  "gene": "UniProtKB:Q9BX26",
  "gene_name": "Synaptonemal complex protein 2",
  "term_id": "GO:0000800",
  "gene_symbol": "SYCP2"
}